{
  "gene_symbol": "UNQ5830/PRO19650/PRO19816",
  "gene": "UniProtKB:Q6UY13",
  "term_label": "positive regulation of extrinsic apoptotic signaling pathway",
  "gene_name": "Putative uncharacterized protein UNQ5830_PRO19650_PRO19816",
  "term_id": "GO:2001238"
}